lysosomal HOPS complex [GO:1902501] (cellular component) Definition: Any HOPS complex that is part of a lysosomal membrane. References: PMID:23645161 Sources: GOC:TermGenie Also known as: lysosomal membrane HOPS complex Relationships: is a type of vacuolar HOPS complex [GO:1902500]; is part of lysosomal membrane [GO:0005765]